rebaudioside B glucosyltransferase activity [GO:0102382] (MF) Relationships: is a type of GO:0016758 Sources: RHEA:61760 Definition: Catalysis of the reaction: rebaudioside B + UDP-alpha-D-glucose = rebaudioside A + UDP.